N5-(carboxyethyl)ornithine synthase activity [GO:0047126] (molecular function) Sources: EC:1.5.1.24, RHEA:18661 Also known as: 5-N-(L-1-carboxyethyl)-L-ornithine:NADP+ oxidoreductase (L-ornithine-forming), N5-(L-1-carboxyethyl)-L-ornithine:NADP+ oxidoreductase (L-ornithine-forming) Definition: Catalysis of the reaction: N(5)-[1(S)-1-carboxyethyl]-L-ornithine + H2O + NADP+ = L-ornithine + H+ + NADPH + pyruvate. Relationships: is a type of GO:0016646